central nervous system structural organization [GO:0021597] (biological process) Relationships: is a type of anatomical structure arrangement [GO:0048532]; is part of GO:0021551 Also known as: central nervous system structural organisation Definition: The process that contributes to the act of creating the structural organization of the central nervous system structure. The central nervous system is the core nervous system that serves an integrating and coordinating function. In vertebrates it consists of the brain, spinal cord and spinal nerves. In those invertebrates with a central nervous system it typically consists of a brain, cerebral ganglia and a nerve cord. Sources: GOC:cls, GOC:dgh, GOC:dph, GOC:jid, GO_REF:0000021